iron-sulfur cluster transmembrane transport [GO:1902497] (biological process) Subtypes: iron-sulfur cluster export from the mitochondrion [GO:0140466] Relationships: is a type of iron ion transmembrane transport [GO:0034755]; is a type of GO:1901678 References: PMID:19810706 Sources: GOC:TermGenie, GOC:dph Definition: A process in which an iron-sulfur cluster is transported from one side of a membrane to the other by means of some agent such as a transporter or pore. Also known as: iron-sulfur cluster transport